citrullinase activity [GO:0047781] (molecular function) Relationships: is_a hydrolase activity, acting on carbon-nitrogen (but not peptide) bonds, in linear amides [GO:0016811] Definition: Catalysis of the reaction: H2O + citrulline = NH3 + CO2 + L-ornithine. Sources: EC:3.5.1.20, MetaCyc:CITRULLINASE-RXN Also known as: L-citrulline 5-N-carbamoyldihydrolase activity, L-citrulline N5-carbamoyldihydrolase activity, citrulline hydrolase activity, citrulline ureidase activity